{
  "term_label": "metaphase chromosome alignment",
  "gene": "UniProtKB:Q9NQS7",
  "gene_name": "Inner centromere protein",
  "term_id": "GO:0051310",
  "gene_symbol": "INCENP"
}